{
  "gene": "UniProtKB:A1Z1Q3",
  "gene_name": "ADP-ribose glycohydrolase MACROD2",
  "gene_symbol": "MACROD2",
  "term_id": "GO:0006974",
  "term_label": "DNA damage response"
}